B cell activation involved in immune response [GO:0002312] (biological process) Sources: GOC:jal Also known as: B cell activation during immune response, B lymphocyte activation during immune response, B-cell activation during immune response, B-lymphocyte activation during immune response Relationships: is_a lymphocyte activation involved in immune response [GO:0002285]; is a type of GO:0042113 Subtypes: mature B cell differentiation involved in immune response [GO:0002313], B cell proliferation involved in immune response [GO:0002322], isotype switching [GO:0045190] Definition: The change in morphology and behavior of a mature or immature B cell during an immune response, resulting from exposure to a mitogen, cytokine, chemokine, cellular ligand, or an antigen for which it is specific.